{
  "gene_name": "Nucleotide-binding oligomerization domain-containing protein 2",
  "term_label": "response to muramyl dipeptide",
  "gene_symbol": "NOD2",
  "term_id": "GO:0032495",
  "gene": "UniProtKB:Q9HC29"
}